{
  "term_label": "Unknown biological process",
  "term_id": "UNKNOWN:0002",
  "gene_name": "Reticulocalbin-1",
  "gene_symbol": "RCN1",
  "gene": "UniProtKB:Q15293"
}